{
  "gene": "UniProtKB:A0A0B4J2B6",
  "term_label": "antigen binding",
  "gene_name": "Immunoglobulin heavy variable 2_OR16-5 (non-functional) (Fragment)",
  "gene_symbol": "IGHV2OR16-5",
  "term_id": "GO:0003823"
}